{
  "gene_name": "E3 ubiquitin-protein ligase rififylin",
  "term_id": "GO:0043161",
  "term_label": "proteasome-mediated ubiquitin-dependent protein catabolic process",
  "gene": "UniProtKB:Q8WZ73",
  "gene_symbol": "RFFL"
}